{
  "gene": "UniProtKB:P55290",
  "term_id": "GO:0044331",
  "gene_name": "Cadherin-13",
  "gene_symbol": "CDH13",
  "term_label": "cell-cell adhesion mediated by cadherin"
}